{
  "term_id": "UNKNOWN:0002",
  "gene_name": "RNA-binding protein 43",
  "gene": "UniProtKB:Q6ZSC3",
  "term_label": "Unknown biological process",
  "gene_symbol": "RBM43"
}